{
  "term_id": "GO:0016485",
  "gene_symbol": "HPN",
  "gene_name": "Serine protease hepsin",
  "term_label": "protein processing",
  "gene": "UniProtKB:P05981"
}